chemokine (C-C motif) ligand 17 production [GO:0044809] (biological process) Also known as: CCL17 production, TARC production, thymus and activation regulated chemokine production Relationships: is a type of chemokine production [GO:0032602] Definition: The appearance of chemokine (C-C motif) ligand 17 (CCL17) due to biosynthesis or secretion following a cellular stimulus, resulting in an increase in its intracellular or extracellular levels. Sources: GOC:rv